{
  "gene": "UniProtKB:Q17RG1",
  "gene_name": "BTB_POZ domain-containing protein KCTD19",
  "term_id": "UNKNOWN:0002",
  "gene_symbol": "KCTD19",
  "term_label": "Unknown biological process"
}